{
  "gene": "UniProtKB:Q6PHR2",
  "term_id": "GO:0000045",
  "gene_name": "Serine_threonine-protein kinase ULK3",
  "term_label": "autophagosome assembly",
  "gene_symbol": "ULK3"
}